{
  "term_id": "GO:0043161",
  "gene_symbol": "KBTBD12",
  "gene_name": "Kelch repeat and BTB domain-containing protein 12",
  "term_label": "proteasome-mediated ubiquitin-dependent protein catabolic process",
  "gene": "UniProtKB:Q3ZCT8"
}